response to endothelin [GO:1990839] (biological process) Relationships: is a type of response to peptide hormone [GO:0043434] Subtypes: cellular response to endothelin [GO:1990859] References: PMID:16365184 Definition: Any process that results in a change in state or activity of a cell or an organism (in terms of movement, secretion, enzyme production, gene expression, etc.) as a result of an endothelin stimulus. Endothelin is any of three secretory vasoconstrictive peptides (endothelin-1, -2, -3).